negative regulation of mitotic sister chromatid segregation [GO:0033048] (biological process) Definition: Any process that stops, prevents, or reduces the frequency, rate or extent of sister chromatid segregation during mitosis. Sources: GOC:mah Relationships: is a type of GO:0033046; is a type of regulation of mitotic sister chromatid segregation [GO:0033047]; negatively regulates mitotic sister chromatid segregation [GO:0000070] Subtypes: negative regulation of mitotic sister chromatid separation [GO:2000816]